dol-P-Man:Man(6)GlcNAc(2)-PP-Dol alpha-1,2-mannosyltransferase activity [GO:0052926] (molecular function) Relationships: is a type of alpha-1,2-mannosyltransferase activity [GO:0000026]; is a type of GO:0120562 Definition: Catalysis of the reaction: an alpha-D-Man-(1->2)-alpha-D-Man-(1->2)-alpha-D-Man-(1->3)-[alpha-D-Man-(1->3)-alpha-D-Man-(1->6)]-beta-D-Man-(1->4)-beta-D-GlcNAc-(1->4)-alpha-D-GlcNAc-diphospho-di-trans,poly-cis-dolichol + a di-trans,poly-cis-dolichyl beta-D-mannosyl phosphate = an alpha-D-Man-(1->2)-alpha-D-Man-(1->2)-alpha-D-Man-(1->3)-[alpha-D-Man-(1->2)-alpha-D-Man-(1->3)-alpha-D-Man-(1->6)]-beta-D-Man-(1->4)-beta-D-GlcNAc-(1->4)-alpha-D-GlcNAc-diphospho-di-trans,poly-cis-dolichol + a di-trans,poly-cis-dolichyl phosphate + H+. Also known as: dolichylphosphomannose-dependent ALG9 mannosyltransferase activity Sources: RHEA:29531